{
  "term_id": "UNKNOWN:0001",
  "gene": "UniProtKB:P49721",
  "term_label": "Unknown molecular function",
  "gene_symbol": "PSMB2",
  "gene_name": "Proteasome subunit beta type-2"
}